{
  "term_label": "mRNA binding",
  "gene_symbol": "LARP6",
  "gene_name": "La-related protein 6",
  "term_id": "GO:0003729",
  "gene": "UniProtKB:Q9BRS8"
}